{
  "term_label": "calcium/calmodulin-dependent protein kinase activity",
  "gene": "UniProtKB:Q8IU85",
  "term_id": "GO:0004683",
  "gene_symbol": "CAMK1D",
  "gene_name": "Calcium_calmodulin-dependent protein kinase type 1D"
}